{
  "gene_name": "Polyunsaturated fatty acid lipoxygenase ALOX15B",
  "term_label": "lipid oxidation",
  "term_id": "GO:0034440",
  "gene": "UniProtKB:O15296",
  "gene_symbol": "ALOX15B"
}